{
  "term_id": "GO:0005886",
  "gene_name": "Solute carrier family 52, riboflavin transporter, member 3",
  "gene_symbol": "SLC52A3",
  "term_label": "plasma membrane",
  "gene": "UniProtKB:Q9NQ40"
}